{
  "term_id": "UNKNOWN:0002",
  "gene_name": "Putative uncharacterized protein LOC401522",
  "term_label": "Unknown biological process",
  "gene_symbol": "Q5VSD8",
  "gene": "UniProtKB:Q5VSD8"
}